{
  "term_label": "nucleus",
  "term_id": "GO:0005634",
  "gene": "UniProtKB:Q92618",
  "gene_symbol": "ZNF516",
  "gene_name": "Zinc finger protein 516"
}